{
  "gene": "UniProtKB:Q8NFL0",
  "gene_symbol": "B3GNT7",
  "term_id": "GO:0018146",
  "term_label": "keratan sulfate proteoglycan biosynthetic process",
  "gene_name": "UDP-GlcNAc:betaGal beta-1,3-N-acetylglucosaminyltransferase 7"
}